histone H4K12ac reader activity [GO:0140011] (MF) Definition: A histone reader that recognizes a histone H4 acetylated at lysine 12. Note: Note that the residue position corresponds to the canonical human H4 histone (UniProtKB:P02309); this residue is conserved across all eukaryotes. Note that the initiation methionine is cleaved, so the first residue is S1. Also known as: H4K12ac modified histone binding References: PMID:14731392 Relationships: is a type of histone H4 reader activity [GO:0140008]